regulation of cardiac muscle cell myoblast differentiation [GO:2000690] (biological process) Also known as: regulation of myocardial precursor cell differentiation, regulation of cardiac myoblast differentiation Sources: GOC:obol Definition: Any process that modulates the frequency, rate or extent of cardiac muscle cell myoblast differentiation. Subtypes: negative regulation of cardiac muscle cell myoblast differentiation [GO:2000691], positive regulation of cardiac muscle cell myoblast differentiation [GO:2000700] Relationships: is a type of regulation of myoblast differentiation [GO:0045661]; is a type of regulation of cardioblast differentiation [GO:0051890]; regulates GO:0060379